{
  "term_label": "Unknown biological process",
  "gene_symbol": "ZMYND12",
  "term_id": "UNKNOWN:0002",
  "gene_name": "Zinc finger MYND domain-containing protein 12",
  "gene": "UniProtKB:Q9H0C1"
}